{
  "term_id": "GO:0016174",
  "gene_name": "NADPH oxidase 4",
  "gene": "UniProtKB:Q9NPH5",
  "term_label": "NAD(P)H oxidase H2O2-forming activity",
  "gene_symbol": "NOX4"
}